symbiont-mediated perturbation of host cell cycle G1/S transition checkpoint [GO:0039645] (biological process) Definition: A process in which a symbiont interferes with the normal execution of the host cell G1/S transition checkpoint. The host is defined as the larger of the organisms involved in a symbiotic interaction. References: PMID:24501404 Sources: VZ:880 Also known as: G1/S host cell cycle checkpoint dysregulation by virus, perturbation by virus of host G1/S transition checkpoint, modulation by virus of host G1/S transition checkpoint Relationships: is a type of GO:0044071